{
  "gene_name": "Notch homolog 2 N-terminal-like protein R",
  "term_label": "Unknown molecular function",
  "term_id": "UNKNOWN:0001",
  "gene": "UniProtKB:A0A096LNW5",
  "gene_symbol": "NOTCH2NLR"
}